{
  "gene_symbol": "DCBLD2",
  "gene_name": "Discoidin, CUB and LCCL domain-containing protein 2",
  "term_id": "GO:0038023",
  "gene": "UniProtKB:Q96PD2",
  "term_label": "signaling receptor activity"
}